{
  "gene_symbol": "DDRGK1",
  "term_label": "ubiquitin-like protein ligase binding",
  "term_id": "GO:0044389",
  "gene": "UniProtKB:Q96HY6",
  "gene_name": "DDRGK domain-containing protein 1"
}